{
  "gene": "UniProtKB:A0A0B4J2B5",
  "gene_symbol": "IGHV3OR16-9",
  "term_id": "GO:0003823",
  "term_label": "antigen binding",
  "gene_name": "Immunoglobulin heavy variable 3_OR16-9 (non-functional) (Fragment)"
}